{
  "term_label": "extracellular exosome",
  "gene_symbol": "GPRC5A",
  "gene_name": "Retinoic acid-induced protein 3",
  "term_id": "GO:0070062",
  "gene": "UniProtKB:Q8NFJ5"
}